{
  "gene_symbol": "DERL3",
  "gene": "UniProtKB:Q96Q80",
  "term_label": "ERAD pathway",
  "term_id": "GO:0036503",
  "gene_name": "Derlin-3"
}